{
  "term_label": "immune response",
  "term_id": "GO:0006955",
  "gene": "UniProtKB:A0A0A6YYC5",
  "gene_name": "T cell receptor alpha variable 14_delta variable 4",
  "gene_symbol": "TRAV14DV4"
}